{
  "gene_symbol": "PRSS46P",
  "gene_name": "Putative serine protease 46",
  "term_label": "Unknown cellular component",
  "term_id": "UNKNOWN:0003",
  "gene": "UniProtKB:E5RG02"
}